intraglomerular mesangial cell proliferation [GO:0072123] (BP) Definition: The multiplication or reproduction of intraglomerular glomerular mesangium cells by cell division, resulting in the expansion of their population. Intraglomerular mesangial cells are specialized pericytes located among the glomerular capillaries within a renal corpuscle of a kidney. They are required for filtration, structural support and phagocytosis. Subtypes: mesonephric intraglomerular mesangial cell proliferation [GO:0061270], metanephric intraglomerular mesangial cell proliferation [GO:0072263] Sources: GOC:mtg_kidney_jan10 Relationships: is_a GO:0072110